negative regulation of mitotic cell cycle DNA replication [GO:1903464] (biological process) Relationships: is a type of negative regulation of mitotic cell cycle [GO:0045930]; is a type of negative regulation of nuclear cell cycle DNA replication [GO:1902576]; is a type of GO:1903463; negatively regulates mitotic DNA replication [GO:1902969] References: PMID:1234 Sources: GOC:TermGenie, GOC:mtg_cell_cycle, GO_REF:0000058 Subtypes: negative regulation of mitotic DNA replication initiation [GO:1903467] Definition: Any process that stops, prevents or reduces the frequency, rate or extent of mitotic cell cycle DNA replication. Also known as: down regulation of DNA replication involved in S phase involved in mitotic cell cycle, down regulation of DNA replication involved in S-phase involved in mitotic cell cycle, down regulation of mitotic cell cycle DNA replication, down regulation of mitotic nuclear cell cycle DNA replication, down-regulation of DNA replication involved in S phase involved in mitotic cell cycle, down-regulation of DNA replication involved in S-phase involved in mitotic cell cycle, down-regulation of mitotic cell cycle DNA replication, down-regulation of mitotic nuclear cell cycle DNA replication, downregulation of DNA replication involved in S phase involved in mitotic cell cycle, downregulation of DNA replication involved in S-phase involved in mitotic cell cycle, downregulation of mitotic cell cycle DNA replication, downregulation of mitotic nuclear cell cycle DNA replication, negative regulation of DNA replication involved in S phase involved in mitotic cell cycle, negative regulation of DNA replication involved in S-phase involved in mitotic cell cycle, negative regulation of mitotic nuclear cell cycle DNA replication, inhibition of DNA replication involved in S phase involved in mitotic cell cycle, inhibition of DNA replication involved in S-phase involved in mitotic cell cycle, inhibition of mitotic cell cycle DNA replication, inhibition of mitotic nuclear cell cycle DNA replication, down regulation of DNA replication during S phase involved in mitotic cell cycle, down regulation of nuclear cell cycle DNA replication involved in mitotic cell cycle, down-regulation of DNA replication during S phase involved in mitotic cell cycle, down-regulation of nuclear cell cycle DNA replication involved in mitotic cell cycle, downregulation of DNA replication during S phase involved in mitotic cell cycle, downregulation of nuclear cell cycle DNA replication involved in mitotic cell cycle, inhibition of DNA replication during S phase involved in mitotic cell cycle, inhibition of nuclear cell cycle DNA replication involved in mitotic cell cycle, negative regulation of DNA replication during S phase involved in mitotic cell cycle, negative regulation of nuclear cell cycle DNA replication involved in mitotic cell cycle